{
  "term_label": "myosin II complex",
  "gene_name": "Myosin-3",
  "gene_symbol": "MYH3",
  "term_id": "GO:0016460",
  "gene": "UniProtKB:P11055"
}